regulation of nervous system process [GO:0031644] (biological process) Also known as: regulation of neurological process, regulation of neurological system process, regulation of neurophysiological process Sources: GOC:dph, GOC:mah, GOC:tb Subtypes: negative regulation of nervous system process [GO:0031645], positive regulation of nervous system process [GO:0031646], regulation of sensory perception [GO:0051931], GO:0051969, regulation of olfactory learning [GO:0090328], modulation of excitatory postsynaptic potential [GO:0098815], GO:0098828 Definition: Any process that modulates the frequency, rate or extent of a neurophysiological process, an organ system process carried out by any of the organs or tissues of the nervous system. Relationships: is a type of regulation of system process [GO:0044057]; regulates GO:0050877